{
  "gene": "UniProtKB:P04114",
  "term_label": "cholesterol homeostasis",
  "term_id": "GO:0042632",
  "gene_name": "Apolipoprotein B-100",
  "gene_symbol": "APOB"
}